{
  "term_label": "neuronal cell body",
  "gene_name": "BMP_retinoic acid-inducible neural-specific protein 2",
  "gene": "UniProtKB:Q9C0B6",
  "gene_symbol": "BRINP2",
  "term_id": "GO:0043025"
}